{
  "gene_name": "Amelotin",
  "term_id": "GO:0070175",
  "gene_symbol": "AMTN",
  "gene": "UniProtKB:Q6UX39",
  "term_label": "positive regulation of enamel mineralization"
}